{
  "gene": "UniProtKB:P05111",
  "gene_name": "Inhibin alpha chain",
  "term_label": "cytokine activity",
  "gene_symbol": "INHA",
  "term_id": "GO:0005125"
}